{
  "gene": "UniProtKB:O75152",
  "term_id": "GO:0005634",
  "gene_name": "Zinc finger CCCH domain-containing protein 11A",
  "gene_symbol": "ZC3H11A",
  "term_label": "nucleus"
}